{
  "gene_symbol": "C1orf105",
  "term_id": "UNKNOWN:0003",
  "term_label": "Unknown cellular component",
  "gene_name": "Uncharacterized protein C1orf105",
  "gene": "UniProtKB:O95561"
}